imaginal disc development [GO:0007444] (biological process) Definition: The process whose specific outcome is the progression of the imaginal disc over time, from its formation to the metamorphosis to form adult structures. Imaginal discs are epithelial infoldings in the larvae of holometabolous insects that develop into adult structures (legs, antennae, wings, etc.). Relationships: is a type of animal organ development [GO:0048513] Sources: GOC:bf, ISBN:0879694238 Subtypes: clypeo-labral disc development [GO:0035213], eye-antennal disc development [GO:0035214], genital disc development [GO:0035215], haltere disc development [GO:0035216], labial disc development [GO:0035217], GO:0035218, prothoracic disc development [GO:0035219], wing disc development [GO:0035220]